{
  "gene_name": "Dual specificity protein kinase CLK2",
  "term_id": "GO:0005634",
  "gene_symbol": "CLK2",
  "term_label": "nucleus",
  "gene": "UniProtKB:P49760"
}